{
  "term_id": "GO:0048812",
  "gene": "UniProtKB:Q96NW4",
  "gene_name": "Ankyrin repeat domain-containing protein 27",
  "gene_symbol": "ANKRD27",
  "term_label": "neuron projection morphogenesis"
}